{
  "term_label": "antigen binding",
  "gene_name": "Immunoglobulin heavy variable 3-11",
  "gene": "UniProtKB:P01762",
  "term_id": "GO:0003823",
  "gene_symbol": "IGHV3-11"
}